{
  "gene": "UniProtKB:P52926",
  "term_id": "GO:0035556",
  "term_label": "intracellular signal transduction",
  "gene_name": "High mobility group protein HMGI-C",
  "gene_symbol": "HMGA2"
}